{
  "term_id": "GO:0000423",
  "term_label": "mitophagy",
  "gene_name": "Autophagy-related protein 13",
  "gene_symbol": "ATG13",
  "gene": "UniProtKB:O75143"
}